{
  "gene_symbol": "KLK15",
  "gene": "UniProtKB:Q9H2R5",
  "term_id": "GO:0030141",
  "term_label": "secretory granule",
  "gene_name": "Kallikrein-15"
}